{
  "term_label": "late endosome to vacuole transport",
  "term_id": "GO:0045324",
  "gene_name": "Charged multivesicular body protein 1a",
  "gene_symbol": "CHMP1A",
  "gene": "UniProtKB:Q9HD42"
}